tissue kallikrein-kinin cascade [GO:0002255] (biological process) Definition: A series of reactions that takes place outside the cell initiated by the action of tissue (glandular) kallikreins on low molecular weight kininogen in response to tissue damage. Tissue kallikreins are present in glandular tissues and their fluids, such as the salivary glands, sweat glands, pancreas, and kidney. The ultimate products of the tissue kallikrein-kinin cascade include kallidin and bradykinin, agents known to induce smooth muscle contraction, vasoconstriction, and increased vascular permeability. References: PMID:11842287, PMID:14501145 Sources: GOC:add Relationships: is a type of kinin cascade [GO:0002254] Also known as: glandular kallikrein-kinin cascade Regulation: regulated by regulation of tissue kallikrein-kinin cascade [GO:0002382]; negatively regulated by negative regulation of tissue kallikrein-kinin cascade [GO:0002546]; positively regulated by positive regulation of tissue kallikrein-kinin cascade [GO:0002547]